{
  "term_label": "Unknown biological process",
  "gene_name": "Tripeptidyl-peptidase 2",
  "gene_symbol": "TPP2",
  "gene": "UniProtKB:P29144",
  "term_id": "UNKNOWN:0002"
}